{
  "gene_name": "Aldo-keto reductase family 1 member C2",
  "gene": "UniProtKB:P52895",
  "term_label": "bile acid binding",
  "term_id": "GO:0032052",
  "gene_symbol": "AKR1C2"
}